{
  "term_id": "GO:0005829",
  "gene_symbol": "HSPA7",
  "term_label": "cytosol",
  "gene": "UniProtKB:P48741",
  "gene_name": "Putative heat shock 70 kDa protein 7"
}